{
  "gene_symbol": "SERPINB3",
  "term_id": "GO:0005615",
  "gene_name": "Serpin B3",
  "term_label": "extracellular space",
  "gene": "UniProtKB:P29508"
}